{
  "term_label": "calcium-dependent phospholipid binding",
  "gene_name": "Copine-7",
  "term_id": "GO:0005544",
  "gene": "UniProtKB:Q9UBL6",
  "gene_symbol": "CPNE7"
}